epithelium-like organization [GO:0140509] (biological process) References: PMID:21393547, PMID:22902739 Definition: The organization of a polarized cell layer during morphogenesis in protozoa; an example is found during culmination in D. discoideum, involving alpha and beta catenins. Relationships: is a type of anatomical structure morphogenesis [GO:0009653]